{
  "gene_name": "Advanced glycosylation end product-specific receptor",
  "gene": "UniProtKB:Q15109",
  "gene_symbol": "AGER",
  "term_id": "GO:0005615",
  "term_label": "extracellular space"
}